{
  "gene": "UniProtKB:Q9UN88",
  "gene_name": "Gamma-aminobutyric acid receptor subunit theta",
  "term_label": "GABA-A receptor activity",
  "gene_symbol": "GABRQ",
  "term_id": "GO:0004890"
}